{
  "term_id": "GO:0000932",
  "gene": "UniProtKB:Q8IUX4",
  "gene_name": "DNA dC-dU-editing enzyme APOBEC-3F",
  "term_label": "P-body",
  "gene_symbol": "APOBEC3F"
}